cGMP-dependent protein kinase activity [GO:0004692] (molecular function) Note: This reaction requires the presence of cGMP. Relationships: is a type of GO:0004690; has part cGMP binding [GO:0030553] Sources: GOC:mah Also known as: 3':5'-cyclic GMP-dependent protein kinase activity, ATP:protein phosphotransferase (cGMP-dependent) activity, PKG, PKG 1alpha, PKG 1beta, PKG II, STK23, cGMP-dependent protein kinase ibeta activity, guanosine 3':5'-cyclic monophosphate-dependent protein kinase activity Definition: cGMP dependent catalysis of the reaction: ATP + a protein = ADP + a phosphoprotein.